{
  "term_label": "microtubule binding",
  "gene_name": "Dystonin",
  "gene_symbol": "DST",
  "term_id": "GO:0008017",
  "gene": "UniProtKB:Q03001"
}